{
  "gene_name": "Spectrin beta chain, erythrocytic",
  "gene": "UniProtKB:P11277",
  "term_id": "GO:0030054",
  "gene_symbol": "SPTB",
  "term_label": "cell junction"
}